maternal-to-zygotic transition of gene expression [GO:0160021] (BP) Definition: Any process that modulates the frequency, rate or extent of gene expression by which developmental control passes from the maternal genome to the zygotic genome. Also known as: MZT References: PMID:19204068, PMID:32558204 Relationships: is a type of regulation of gene expression [GO:0010468]